{
  "term_id": "GO:0005764",
  "gene_symbol": "CTSC",
  "gene": "UniProtKB:P53634",
  "term_label": "lysosome",
  "gene_name": "Dipeptidyl peptidase 1"
}